{
  "term_label": "peptide metabolic process",
  "gene": "UniProtKB:P14384",
  "term_id": "GO:0006518",
  "gene_symbol": "CPM",
  "gene_name": "Carboxypeptidase M"
}